{
  "term_id": "GO:0005615",
  "term_label": "extracellular space",
  "gene_name": "Fibroleukin",
  "gene_symbol": "FGL2",
  "gene": "UniProtKB:Q14314"
}